{
  "term_label": "nucleus",
  "gene_name": "RNA exonuclease 5",
  "term_id": "GO:0005634",
  "gene": "UniProtKB:Q96IC2",
  "gene_symbol": "REXO5"
}